{
  "term_id": "GO:0030574",
  "term_label": "collagen catabolic process",
  "gene_symbol": "MMP19",
  "gene_name": "Matrix metalloproteinase-19",
  "gene": "UniProtKB:Q99542"
}